methanofuran metabolic process [GO:2001119] (biological process) Sources: GOC:mengo_curators Definition: The chemical reactions and pathways involving a methanofuran. Also known as: methanofuran metabolism Subtypes: methanofuran biosynthetic process [GO:2001120] Relationships: is a type of metabolic process [GO:0008152]